{
  "gene_symbol": "MDK",
  "gene_name": "Midkine",
  "term_label": "Unknown biological process",
  "term_id": "UNKNOWN:0002",
  "gene": "UniProtKB:P21741"
}